{
  "gene_symbol": "GH2",
  "gene": "UniProtKB:P01242",
  "gene_name": "Growth hormone variant",
  "term_id": "GO:0008083",
  "term_label": "growth factor activity"
}